{
  "term_label": "nucleus",
  "gene": "UniProtKB:Q6IQ32",
  "term_id": "GO:0005634",
  "gene_name": "Activity-dependent neuroprotector homeobox protein 2",
  "gene_symbol": "ADNP2"
}